plasma membrane fusion [GO:0045026] (biological process) Relationships: is a type of plasma membrane organization [GO:0007009]; is a type of membrane fusion [GO:0061025] Also known as: cell fusion, cell-cell fusion Definition: The joining of the lipid bilayer membrane that surround a cell with that of another cell, producing a single cell. Sources: GOC:elh, GOC:mtg_muscle Subtypes: fusion of sperm to egg plasma membrane involved in single fertilization [GO:0007342], plasma membrane fusion involved in cytogamy [GO:0032220], fusion of sperm to egg plasma membrane involved in double fertilization forming two zygotes [GO:0061935], GO:0061936